GCG codon-amino acid adaptor activity [GO:0033456] (molecular function) Also known as: alanine tRNA Note: Note that in the standard genetic code, GCG codes for alanine. Definition: A triplet codon-amino acid adaptor activity that recognizes a GCG codon. Relationships: is a type of triplet codon-amino acid adaptor activity [GO:0030533] Sources: GOC:mah